{
  "gene_name": "mRNA-decapping enzyme 1A",
  "gene_symbol": "DCP1A",
  "term_label": "deadenylation-dependent decapping of nuclear-transcribed mRNA",
  "gene": "UniProtKB:Q9NPI6",
  "term_id": "GO:0000290"
}